cellular response to ketone [GO:1901655] (biological process) Definition: Any process that results in a change in state or activity of a cell (in terms of movement, secretion, enzyme production, gene expression, etc.) as a result of a ketone stimulus. Sources: GOC:TermGenie, GOC:pr Subtypes: cellular response to vitamin K [GO:0071307], cellular response to prostaglandin E stimulus [GO:0071380], cellular response to corticosterone stimulus [GO:0071386], cellular response to cortisol stimulus [GO:0071387], cellular response to cortisone stimulus [GO:0071388], GO:0071390, cellular response to progesterone stimulus [GO:0071393], GO:0071394, cellular response to cycloheximide [GO:0071409], cellular response to hydroxyisoflavone [GO:0071413], cellular response to dexamethasone stimulus [GO:0071549], cellular response to prostaglandin D stimulus [GO:0071799], cellular response to tetracycline [GO:0072746], cellular response to rapamycin [GO:0072752], cellular response to methylglyoxal [GO:0097238], GO:1902709, cellular response to differentiation-inducing factor 1 [GO:1903014], cellular response to dehydroepiandrosterone [GO:1903495], cellular response to 11-deoxycorticosterone [GO:1903497], cellular response to aldosterone [GO:1904045], cellular response to forskolin [GO:1904322], cellular response to nocodazole [GO:1904403], cellular response to wortmannin [GO:1904568], cellular response to phorbol 13-acetate 12-myristate [GO:1904628], cellular response to curcumin [GO:1904644], GO:1904648, cellular response to haloperidol [GO:1905120] Relationships: is_a response to ketone [GO:1901654]; is a type of cellular response to oxygen-containing compound [GO:1901701]